2-methyl-6-solanyl-1,4-benzoquinone methyltransferase activity [GO:0051742] (molecular function) Sources: MetaCyc:RXN-2762 Also known as: MSBQ methyltransferase activity Definition: Catalysis of the reaction: 2-methyl-6-solanyl-1,4-benzoquinone + S-adenosyl-methionine = 2,3-dimethyl-6-solanyl-1,4-benzoquinone + S-adenosyl-homocysteine. Relationships: is a type of S-adenosylmethionine-dependent methyltransferase activity [GO:0008757]